{
  "gene_symbol": "GAGE12I",
  "gene": "UniProtKB:P0CL82",
  "term_id": "UNKNOWN:0002",
  "gene_name": "G antigen 12I",
  "term_label": "Unknown biological process"
}